{
  "gene": "UniProtKB:Q9ULJ7",
  "term_label": "Unknown molecular function",
  "gene_name": "Ankyrin repeat domain-containing protein 50",
  "gene_symbol": "ANKRD50",
  "term_id": "UNKNOWN:0001"
}